{
  "term_label": "Unknown cellular component",
  "gene": "UniProtKB:Q16825",
  "term_id": "UNKNOWN:0003",
  "gene_name": "Tyrosine-protein phosphatase non-receptor type 21",
  "gene_symbol": "PTPN21"
}